{
  "term_label": "RNA polymerase II cis-regulatory region sequence-specific DNA binding",
  "gene_symbol": "TFCP2L1",
  "gene": "UniProtKB:Q9NZI6",
  "term_id": "GO:0000978",
  "gene_name": "Transcription factor CP2-like protein 1"
}